{
  "gene_name": "Adenosine receptor A3",
  "gene": "UniProtKB:P0DMS8",
  "term_id": "GO:0030425",
  "term_label": "dendrite",
  "gene_symbol": "ADORA3"
}